{
  "gene_symbol": "PHGR1",
  "term_label": "Unknown cellular component",
  "term_id": "UNKNOWN:0003",
  "gene_name": "Proline, histidine and glycine-rich protein 1",
  "gene": "UniProtKB:C9JFL3"
}